{
  "gene_symbol": "CD86",
  "gene_name": "T-lymphocyte activation antigen CD86",
  "term_label": "cell surface receptor signaling pathway",
  "gene": "UniProtKB:P42081",
  "term_id": "GO:0007166"
}